{
  "gene_symbol": "ABCC3",
  "term_id": "GO:0016323",
  "gene": "UniProtKB:O15438",
  "gene_name": "ATP-binding cassette sub-family C member 3",
  "term_label": "basolateral plasma membrane"
}